{
  "term_label": "NLRP3 inflammasome complex",
  "term_id": "GO:0072559",
  "gene_name": "Apoptosis-associated speck-like protein containing a CARD",
  "gene_symbol": "PYCARD",
  "gene": "UniProtKB:Q9ULZ3"
}